{
  "gene_name": "Pituitary homeobox 2",
  "term_label": "anatomical structure morphogenesis",
  "gene_symbol": "PITX2",
  "term_id": "GO:0009653",
  "gene": "UniProtKB:Q99697"
}